{
  "term_label": "site of polarized growth",
  "term_id": "GO:0030427",
  "gene_name": "Coactosin-like protein",
  "gene": "UniProtKB:Q14019",
  "gene_symbol": "COTL1"
}